{
  "gene_name": "Manganese-dependent ADP-ribose_CDP-alcohol diphosphatase",
  "term_id": "UNKNOWN:0002",
  "term_label": "Unknown biological process",
  "gene": "UniProtKB:Q3LIE5",
  "gene_symbol": "ADPRM"
}